{
  "gene_name": "Olfactory receptor 6K2",
  "gene": "UniProtKB:Q8NGY2",
  "term_id": "GO:0004984",
  "gene_symbol": "OR6K2",
  "term_label": "olfactory receptor activity"
}